{
  "gene": "UniProtKB:Q96PQ6",
  "term_label": "nucleus",
  "term_id": "GO:0005634",
  "gene_symbol": "ZNF317",
  "gene_name": "Zinc finger protein 317"
}